axon ensheathment in central nervous system [GO:0032291] (biological process) Definition: The process in which a glial cell membrane closes around an axon in the central nervous system. This can be a myelinating or a non-myelinating neuron-glial interaction. Sources: GOC:dgh Also known as: ensheathment of axons in central nervous system Relationships: is a type of GO:0008366 Subtypes: central nervous system myelination [GO:0022010], non-myelinated axon ensheathment in central nervous system [GO:0032293]